{
  "term_label": "Unknown biological process",
  "term_id": "UNKNOWN:0002",
  "gene_symbol": "OR52E5",
  "gene": "UniProtKB:Q8NH55",
  "gene_name": "Olfactory receptor 52E5"
}